2-nitrophenol 2-monooxygenase activity [GO:0047549] (molecular function) Definition: Catalysis of the reaction: 2-nitrophenol + 2 H+ + 2 NADPH + O2 = catechol + H2O + 2 NADP+ + nitrite. Sources: EC:1.14.13.31, RHEA:19457 Also known as: nitrophenol oxygenase activity, 2-nitrophenol oxygenase activity, 2-nitrophenol,NADPH:oxygen 2-oxidoreductase (2-hydroxylating, nitrite-forming) Relationships: is a type of oxidoreductase activity, acting on paired donors, with incorporation or reduction of molecular oxygen, NAD(P)H as one donor, and incorporation of one atom of oxygen [GO:0016709]